{
  "term_label": "translation initiation factor activity",
  "gene_name": "Eukaryotic translation initiation factor 3 subunit L",
  "gene_symbol": "EIF3L",
  "gene": "UniProtKB:Q9Y262",
  "term_id": "GO:0003743"
}